{
  "gene_name": "Inactive tyrosine-protein kinase PRAG1",
  "term_label": "protein kinase activity",
  "gene_symbol": "PRAG1",
  "gene": "UniProtKB:Q86YV5",
  "term_id": "GO:0004672"
}